{
  "term_label": "tumor necrosis factor receptor activity",
  "term_id": "GO:0005031",
  "gene_symbol": "TNFRSF4",
  "gene_name": "Tumor necrosis factor receptor superfamily member 4",
  "gene": "UniProtKB:P43489"
}